{
  "term_label": "cytosol",
  "term_id": "GO:0005829",
  "gene": "UniProtKB:Q6UB35",
  "gene_symbol": "MTHFD1L",
  "gene_name": "Monofunctional C1-tetrahydrofolate synthase, mitochondrial"
}